ATP:3'-cytidine-cytidine-tRNA adenylyltransferase activity [GO:0052929] (molecular function) Relationships: is a type of adenylyltransferase activity [GO:0070566]; is a type of catalytic activity, acting on a tRNA [GO:0140101] Also known as: ATP:tRNA adenylyltransferase activity, ATP:3'-CC-tRNA adenylyltransferase activity Definition: Catalysis of the reaction: a tRNA with a 3' CC end + ATP = a tRNA with a 3' CCA end + diphosphate. References: PMID:31936900, PMID:33095240 Sources: RHEA:60012